{
  "term_label": "nucleus",
  "gene_symbol": "UBL5",
  "gene": "UniProtKB:Q9BZL1",
  "gene_name": "Ubiquitin-like protein 5",
  "term_id": "GO:0005634"
}